{
  "gene_symbol": "RPA4",
  "gene_name": "Replication protein A 30 kDa subunit",
  "term_label": "DNA replication",
  "term_id": "GO:0006260",
  "gene": "UniProtKB:Q13156"
}